regulation of eye photoreceptor cell development [GO:0042478] (BP) Relationships: is a type of regulation of photoreceptor cell differentiation [GO:0046532]; is a type of regulation of cell development [GO:0060284]; regulates GO:0042462 Definition: Any process that modulates the frequency, rate or extent of eye photoreceptor development. Also known as: regulation of eye photoreceptor development Sources: GOC:jl Subtypes: positive regulation of eye photoreceptor cell development [GO:0042479], negative regulation of eye photoreceptor cell development [GO:0042480], regulation of compound eye photoreceptor development [GO:0045314]